{
  "term_id": "GO:0005730",
  "term_label": "nucleolus",
  "gene": "UniProtKB:Q9Y3A2",
  "gene_name": "Probable U3 small nucleolar RNA-associated protein 11",
  "gene_symbol": "UTP11"
}